{
  "gene": "UniProtKB:F5H094",
  "gene_symbol": "SLCO1B3-SLCO1B7",
  "gene_name": "SLCO1B3-SLCO1B7 readthrough transcript protein",
  "term_label": "basolateral plasma membrane",
  "term_id": "GO:0016323"
}